early meiotic recombination nodule assembly [GO:0042139] (biological process) Relationships: is a type of GO:0007146 References: PMID:9334324 Sources: GOC:jl Definition: During meiosis, the aggregation, arrangement and bonding together of strand exchange proteins (recombinases) to form small, electron dense structures in association with meiotic chromosomes during leptotene and zygotene.